{
  "gene_name": "Actin, cytoplasmic 1",
  "term_label": "NuA4 histone acetyltransferase complex",
  "term_id": "GO:0035267",
  "gene": "UniProtKB:P60709",
  "gene_symbol": "ACTB"
}